{
  "gene": "UniProtKB:Q96R08",
  "gene_symbol": "OR5B12",
  "term_id": "UNKNOWN:0003",
  "term_label": "Unknown cellular component",
  "gene_name": "Olfactory receptor 5B12"
}